{
  "gene_name": "ATP-dependent RNA helicase DDX39A",
  "gene": "UniProtKB:O00148",
  "gene_symbol": "DDX39A",
  "term_label": "mRNA splicing, via spliceosome",
  "term_id": "GO:0000398"
}